{
  "term_label": "ubiquitin protein ligase activity",
  "gene_name": "E3 ubiquitin-protein ligase MARCHF1",
  "gene_symbol": "MARCHF1",
  "term_id": "GO:0061630",
  "gene": "UniProtKB:Q8TCQ1"
}